{
  "gene": "UniProtKB:O75437",
  "gene_symbol": "ZNF254",
  "term_label": "regulation of transcription by RNA polymerase II",
  "term_id": "GO:0006357",
  "gene_name": "Zinc finger protein 254"
}